alpha5-beta5-fibronectin-SFRP2 complex [GO:0071138] (cellular component) Definition: A protein complex that consists of an alpha5-beta5 integrin complex bound to fibronectin and secreted frizzled-related protein 2. Also known as: ITGA5-ITGB5-FN-1-SFRP2 complex Relationships: is a type of plasma membrane protein complex [GO:0098797] References: PMID:14709558